{
  "gene_name": "Heat shock protein beta-3",
  "gene_symbol": "HSPB3",
  "term_id": "GO:0016607",
  "term_label": "nuclear speck",
  "gene": "UniProtKB:Q12988"
}